{
  "gene": "UniProtKB:P14136",
  "term_id": "GO:0005882",
  "term_label": "intermediate filament",
  "gene_name": "Glial fibrillary acidic protein",
  "gene_symbol": "GFAP"
}